{
  "term_id": "UNKNOWN:0003",
  "gene_name": "Protein LRATD2",
  "gene_symbol": "LRATD2",
  "term_label": "Unknown cellular component",
  "gene": "UniProtKB:Q96KN1"
}